{
  "term_id": "UNKNOWN:0001",
  "gene": "UniProtKB:Q9NQG6",
  "term_label": "Unknown molecular function",
  "gene_name": "Mitochondrial dynamics protein MIEF1",
  "gene_symbol": "MIEF1"
}